{
  "term_id": "GO:0007098",
  "term_label": "centrosome cycle",
  "gene": "UniProtKB:Q5VU43",
  "gene_symbol": "PDE4DIP",
  "gene_name": "Myomegalin"
}